{
  "gene_symbol": "BPESC1",
  "term_id": "UNKNOWN:0001",
  "gene_name": "Putative BPES syndrome breakpoint region protein",
  "gene": "UniProtKB:Q9GZL8",
  "term_label": "Unknown molecular function"
}